positive regulation of interleukin-16 production [GO:0032739] (BP) Also known as: positive regulation of IL-16 production, up regulation of interleukin-16 production, up-regulation of interleukin-16 production, upregulation of interleukin-16 production, activation of interleukin-16 production, positive regulation of interleukin-16 biosynthetic process, stimulation of interleukin-16 production Definition: Any process that activates or increases the frequency, rate, or extent of interleukin-16 production. Sources: GOC:mah Relationships: is a type of positive regulation of cytokine production [GO:0001819]; is a type of regulation of interleukin-16 production [GO:0032659]; positively regulates interleukin-16 production [GO:0032619]